{
  "gene_name": "Protein MAL2",
  "term_id": "GO:0016020",
  "term_label": "membrane",
  "gene_symbol": "MAL2",
  "gene": "UniProtKB:Q969L2"
}